{
  "gene_symbol": "SRPK1",
  "term_label": "intracellular signal transduction",
  "term_id": "GO:0035556",
  "gene": "UniProtKB:Q96SB4",
  "gene_name": "SRSF protein kinase 1"
}